{
  "gene": "UniProtKB:P12755",
  "term_id": "GO:0000981",
  "term_label": "DNA-binding transcription factor activity, RNA polymerase II-specific",
  "gene_symbol": "SKI",
  "gene_name": "Ski oncogene"
}